{
  "gene_name": "GTPase-activating protein and VPS9 domain-containing protein 1",
  "gene_symbol": "GAPVD1",
  "term_label": "endocytic vesicle",
  "gene": "UniProtKB:Q14C86",
  "term_id": "GO:0030139"
}